{
  "term_id": "GO:0048018",
  "gene_symbol": "IGFBPL1",
  "term_label": "receptor ligand activity",
  "gene_name": "Insulin-like growth factor-binding protein-like 1",
  "gene": "UniProtKB:Q8WX77"
}